{
  "term_label": "ubiquitin-like ligase-substrate adaptor activity",
  "gene_symbol": "SPSB1",
  "gene": "UniProtKB:Q96BD6",
  "gene_name": "SPRY domain-containing SOCS box protein 1",
  "term_id": "GO:1990756"
}